{
  "gene_name": "Huntingtin-interacting protein 1",
  "gene_symbol": "HIP1",
  "gene": "UniProtKB:O00291",
  "term_id": "GO:0045742",
  "term_label": "positive regulation of epidermal growth factor receptor signaling pathway"
}